{
  "term_id": "GO:0008277",
  "gene_symbol": "ZDHHC7",
  "gene": "UniProtKB:Q9NXF8",
  "gene_name": "Palmitoyltransferase ZDHHC7",
  "term_label": "regulation of G protein-coupled receptor signaling pathway"
}